{
  "gene_name": "[3-methyl-2-oxobutanoate dehydrogenase [lipoamide]] kinase, mitochondrial",
  "term_id": "GO:0004740",
  "gene_symbol": "BCKDK",
  "term_label": "pyruvate dehydrogenase (acetyl-transferring) kinase activity",
  "gene": "UniProtKB:O14874"
}